{
  "term_label": "chemorepellent activity",
  "gene_symbol": "NRG1",
  "gene": "UniProtKB:Q02297",
  "gene_name": "Pro-neuregulin-1, membrane-bound isoform",
  "term_id": "GO:0045499"
}